{
  "term_label": "beta-galactosidase activity",
  "gene": "UniProtKB:Q8IW92",
  "gene_name": "Beta-galactosidase-1-like protein 2",
  "term_id": "GO:0004565",
  "gene_symbol": "GLB1L2"
}